{
  "gene_symbol": "PRYP4",
  "gene": "UniProtKB:O14603",
  "term_label": "Unknown cellular component",
  "gene_name": "PTPN13-like protein, Y-linked",
  "term_id": "UNKNOWN:0003"
}